pollen-pistil interaction [GO:0009875] (BP) Also known as: pollen-gynoecium interaction Definition: The interaction between a pollen grain and pistil. References: PMID:27899537 Subtypes: pollen-stigma interaction [GO:0140301], GO:0140302 Relationships: is a type of cell communication [GO:0007154]; is part of pollination [GO:0009856]